{
  "term_id": "GO:0005634",
  "gene_name": "Tesmin",
  "term_label": "nucleus",
  "gene": "UniProtKB:Q9Y4I5",
  "gene_symbol": "TESMIN"
}